{
  "term_label": "cilium",
  "term_id": "GO:0005929",
  "gene_name": "ELMO domain-containing protein 3",
  "gene": "UniProtKB:Q96FG2",
  "gene_symbol": "ELMOD3"
}